positive regulation of innate immune response [GO:0045089] (biological process) Definition: Any process that activates or increases the frequency, rate or extent of the innate immune response, the organism's first line of defense against infection. Relationships: is a type of positive regulation of response to biotic stimulus [GO:0002833]; is a type of positive regulation of defense response [GO:0031349]; is a type of positive regulation of response to external stimulus [GO:0032103]; is a type of GO:0045088; is a type of GO:0050778; positively regulates innate immune response [GO:0045087] Sources: GOC:ebc Subtypes: positive regulation of complement activation, lectin pathway [GO:0001870], activation of innate immune response [GO:0002218], GO:0002717, GO:0034052, positive regulation of melanization defense response [GO:0035008], GO:0045958, positive regulation of respiratory burst involved in inflammatory response [GO:0060265], GO:0060332, positive regulation of type I interferon-mediated signaling pathway [GO:0060340], positive regulation of pattern recognition receptor signaling pathway [GO:0062208], GO:1904250, GO:1905036, GO:1905682 Also known as: up regulation of innate immune response, up-regulation of innate immune response, upregulation of innate immune response, stimulation of innate immune response